positive regulation of heptasaccharide transport [GO:1900296] (biological process) Sources: GOC:TermGenie, GOC:mengo_curators Subtypes: positive regulation of maltoheptaose transport [GO:1900308] Definition: Any process that activates or increases the frequency, rate or extent of heptasaccharide transport. Also known as: up regulation of heptasaccharide transport, up-regulation of heptasaccharide transport, upregulation of heptasaccharide transport, activation of heptasaccharide transport Relationships: is a type of positive regulation of transport [GO:0051050]; is a type of regulation of heptasaccharide transport [GO:1900294]; positively regulates heptasaccharide transport [GO:2001104]